isoprene metabolic process [GO:0043611] (biological process) Also known as: 2-methyl-1,3-butadiene metabolic process, 2-methyl-1,3-butadiene metabolism, hemiterpene metabolic process, hemiterpene metabolism, isoprene metabolism Relationships: is a type of terpene metabolic process [GO:0042214]; is a type of olefin metabolic process [GO:1900673] Definition: The chemical reactions and pathways involving isoprene, C5H8. Subtypes: isoprene biosynthetic process [GO:0043612], isoprene catabolic process [GO:0043613] Sources: GOC:jl